{
  "term_label": "amino acid transmembrane transport",
  "term_id": "GO:0003333",
  "gene_symbol": "SLC7A11",
  "gene_name": "Cystine_glutamate transporter",
  "gene": "UniProtKB:Q9UPY5"
}